{
  "gene_name": "Vacuolar protein sorting-associated protein 52 homolog",
  "term_id": "GO:0007041",
  "gene_symbol": "VPS52",
  "term_label": "lysosomal transport",
  "gene": "UniProtKB:Q8N1B4"
}